{
  "gene_name": "Trafficking protein particle complex subunit 10",
  "term_label": "early endosome to Golgi transport",
  "gene": "UniProtKB:P48553",
  "term_id": "GO:0034498",
  "gene_symbol": "TRAPPC10"
}